{
  "gene_name": "Putative Polycomb group protein ASXL3",
  "gene_symbol": "ASXL3",
  "term_id": "GO:0042975",
  "term_label": "peroxisome proliferator activated receptor binding",
  "gene": "UniProtKB:Q9C0F0"
}